{
  "gene_name": "Leucine-rich repeat-containing protein 14B",
  "term_id": "UNKNOWN:0001",
  "term_label": "Unknown molecular function",
  "gene_symbol": "LRRC14B",
  "gene": "UniProtKB:A6NHZ5"
}